{
  "gene": "UniProtKB:P40425",
  "term_label": "animal organ morphogenesis",
  "term_id": "GO:0009887",
  "gene_name": "Pre-B-cell leukemia transcription factor 2",
  "gene_symbol": "PBX2"
}